actin filament polymerization [GO:0030041] (BP) Regulation: regulated by regulation of actin filament polymerization [GO:0030833]; negatively regulated by negative regulation of actin filament polymerization [GO:0030837]; positively regulated by GO:0030838 Relationships: is a type of actin polymerization or depolymerization [GO:0008154]; is a type of protein polymerization [GO:0051258] Definition: Assembly of actin filaments by the addition of actin monomers to a filament. Sources: GOC:mah Also known as: actin polymerization, actin polymerizing activity